{
  "term_label": "cellular response to glucocorticoid stimulus",
  "gene_symbol": "UGT1A4",
  "gene": "UniProtKB:P22310",
  "gene_name": "UDP-glucuronosyltransferase 1A4",
  "term_id": "GO:0071385"
}